{
  "term_label": "extracellular space",
  "gene_name": "Alpha-amylase 1C",
  "gene": "UniProtKB:P0DTE8",
  "gene_symbol": "AMY1C",
  "term_id": "GO:0005615"
}